{
  "gene_name": "Bone morphogenetic protein receptor type-2",
  "term_id": "GO:0043235",
  "term_label": "receptor complex",
  "gene": "UniProtKB:Q13873",
  "gene_symbol": "BMPR2"
}